NMDA selective glutamate receptor signaling pathway [GO:0098989] (biological process) Sources: GOC:dos, ISBN:9780071120005 Relationships: is a type of ionotropic glutamate receptor signaling pathway [GO:0035235]; has part NMDA glutamate receptor activity [GO:0004972] Definition: The series of molecular signals initiated by glutamate binding to an NMDA-selective glutamate receptor on the surface of the target cell, followed by the movement of ions through a channel in the receptor complex, and ending with the regulation of a downstream cellular process, e.g. transcription.